{
  "term_id": "GO:0007186",
  "gene_name": "P2Y purinoceptor 6",
  "term_label": "G protein-coupled receptor signaling pathway",
  "gene": "UniProtKB:Q15077",
  "gene_symbol": "P2RY6"
}